prenol catabolic process [GO:0016092] (biological process) Also known as: prenol breakdown, prenol catabolism, prenol degradation Relationships: is a type of isoprenoid catabolic process [GO:0008300]; is a type of alcohol catabolic process [GO:0046164]; is a type of olefinic compound catabolic process [GO:0120256] Sources: GOC:go_curators Definition: The chemical reactions and pathways resulting in the breakdown of prenols, isoprenoids of general formula (H-CH2-C(CH3)=CH-CH2-)n-OH, any primary monohydroxy alcohol whose carbon skeleton consists of two or more isoprenoid residues linked head to tail.